{
  "term_label": "RNA polymerase II cis-regulatory region sequence-specific DNA binding",
  "gene_symbol": "FOXD4",
  "gene_name": "Forkhead box protein D4",
  "gene": "UniProtKB:Q12950",
  "term_id": "GO:0000978"
}